{
  "gene": "UniProtKB:Q15700",
  "term_label": "regulation of postsynaptic membrane neurotransmitter receptor levels",
  "term_id": "GO:0099072",
  "gene_name": "Disks large homolog 2",
  "gene_symbol": "DLG2"
}